response to neutral pH [GO:0036176] (biological process) Subtypes: filamentous growth of a population of unicellular organisms in response to neutral pH [GO:0036178], cellular response to neutral pH [GO:0036244] Relationships: is a type of GO:0009268 Sources: GOC:di, Wikipedia:PH Definition: Any process that results in a change in state or activity of a cell or an organism (in terms of movement, secretion, enzyme production, gene expression, etc.) as a result of a neutral pH (pH close to 7) stimulus. pH is a measure of the acidity or basicity of an aqueous solution.